{
  "term_id": "GO:0004888",
  "gene_symbol": "VSTM1",
  "gene": "UniProtKB:Q6UX27",
  "gene_name": "V-set and transmembrane domain-containing protein 1",
  "term_label": "transmembrane signaling receptor activity"
}